{
  "term_label": "Unknown cellular component",
  "term_id": "UNKNOWN:0003",
  "gene": "UniProtKB:Q8N1V8",
  "gene_name": "Uncharacterized protein encoded by LINC01561",
  "gene_symbol": "LINC01561"
}